{
  "gene_name": "F-actin-capping protein subunit alpha-1",
  "term_id": "GO:0051015",
  "gene_symbol": "CAPZA1",
  "gene": "UniProtKB:P52907",
  "term_label": "actin filament binding"
}